{
  "term_id": "GO:0005886",
  "gene": "UniProtKB:Q9NWQ8",
  "gene_symbol": "PAG1",
  "gene_name": "Phosphoprotein associated with glycosphingolipid-enriched microdomains 1",
  "term_label": "plasma membrane"
}